{
  "gene_symbol": "PSAPL1",
  "term_label": "Unknown molecular function",
  "gene": "UniProtKB:Q6NUJ1",
  "gene_name": "Proactivator polypeptide-like 1",
  "term_id": "UNKNOWN:0001"
}